{
  "gene_name": "Palmitoyl-protein thioesterase 1",
  "gene": "UniProtKB:P50897",
  "gene_symbol": "PPT1",
  "term_label": "extracellular region",
  "term_id": "GO:0005576"
}